methanol-CoM methyltransferase complex [GO:0043853] (cellular component) References: PMID:9363780 Also known as: methanol-coenzyme M methyltransferase complex, methanol: CoM methyltransferase complex, methanol: coenzyme M methyltransferase complex, methanol:CoM methyltransferase complex, methanol:coenzyme M methyltransferase complex Definition: A heterotrimeric protein complex composed of a methanol methyltransferase subunit, a corrinoid protein and a methanol-specific corrinoid:coenzyme M methyltransferase subunit. Catalyzes the transfer of a methyl group from methanol to coenzyme M as part of the pathway of methanogenesis from methanol. Relationships: is a type of methyltransferase complex [GO:0034708]